{
  "gene": "UniProtKB:Q86Y79",
  "gene_name": "Peptidyl-tRNA hydrolase",
  "gene_symbol": "PTRH1",
  "term_label": "Unknown biological process",
  "term_id": "UNKNOWN:0002"
}